CCA codon-amino acid adaptor activity [GO:0033423] (molecular function) Note: Note that in the standard genetic code, CCA codes for proline. Relationships: is a type of GO:0030533 Definition: A triplet codon-amino acid adaptor activity that recognizes a CCA codon. Also known as: proline tRNA Sources: GOC:mah